{
  "term_id": "GO:0015866",
  "gene": "UniProtKB:Q6NUK1",
  "gene_name": "Mitochondrial adenyl nucleotide antiporter SLC25A24",
  "term_label": "ADP transport",
  "gene_symbol": "SLC25A24"
}